{
  "gene_name": "C-C motif chemokine 26",
  "gene": "UniProtKB:Q9Y258",
  "term_label": "antimicrobial humoral immune response mediated by antimicrobial peptide",
  "gene_symbol": "CCL26",
  "term_id": "GO:0061844"
}